UDP-N-acetylgalactosamine metabolic process [GO:0019276] (biological process) Sources: GOC:ai Definition: The chemical reactions and pathways involving UDP-N-acetylgalactosamine, a substance composed of N-acetylgalactosamine, a common structural unit of oligosaccharides, in glycosidic linkage with uridine diphosphate. Relationships: is a type of amino sugar metabolic process [GO:0006040]; is a type of nucleotide-sugar metabolic process [GO:0009225] Subtypes: UDP-N-acetylgalactosamine biosynthetic process [GO:0019277] Also known as: UDP-N-acetylgalactosamine metabolism